{
  "gene": "UniProtKB:P56556",
  "term_id": "UNKNOWN:0001",
  "term_label": "Unknown molecular function",
  "gene_name": "NADH dehydrogenase [ubiquinone] 1 alpha subcomplex subunit 6",
  "gene_symbol": "NDUFA6"
}